{
  "gene_name": "Katanin p60 ATPase-containing subunit A-like 1",
  "term_id": "GO:0051013",
  "gene_symbol": "KATNAL1",
  "gene": "UniProtKB:Q9BW62",
  "term_label": "microtubule severing"
}